protein secretion by the type VII secretion system [GO:0044315] (biological process) Definition: The process in which proteins are transferred into the extracellular milieu or directly into host cells, via the type VII protein secretion system. References: PMID:17922044, PMID:19876390 Relationships: is a type of protein secretion [GO:0009306]; is a type of protein transmembrane transport [GO:0071806]